{
  "gene": "UniProtKB:O00479",
  "term_label": "chromatin binding",
  "gene_symbol": "HMGN4",
  "gene_name": "High mobility group nucleosome-binding domain-containing protein 4",
  "term_id": "GO:0003682"
}